{
  "term_id": "UNKNOWN:0003",
  "gene_name": "LysM and putative peptidoglycan-binding domain-containing protein 4",
  "gene_symbol": "LYSMD4",
  "gene": "UniProtKB:Q5XG99",
  "term_label": "Unknown cellular component"
}